{
  "gene": "UniProtKB:Q01628",
  "gene_symbol": "IFITM3",
  "gene_name": "Interferon-induced transmembrane protein 3",
  "term_label": "response to type II interferon",
  "term_id": "GO:0034341"
}